cytotoxic T cell degranulation [GO:0043316] (biological process) Definition: The regulated exocytosis of secretory granules containing preformed mediators such as perforin and granzymes by a cytotoxic T cell. Sources: ISBN:0781735149 Also known as: cytotoxic T cell granule exocytosis, cytotoxic T lymphocyte degranulation, cytotoxic T lymphocyte granule exocytosis, cytotoxic T-cell degranulation, cytotoxic T-cell granule exocytosis, cytotoxic T-lymphocyte degranulation, cytotoxic T-lymphocyte granule exocytosis Relationships: is a type of leukocyte degranulation [GO:0043299]; is part of T cell mediated cytotoxicity [GO:0001913]; is part of T cell activation involved in immune response [GO:0002286] Regulation: regulated by regulation of cytotoxic T cell degranulation [GO:0043317]; negatively regulated by negative regulation of cytotoxic T cell degranulation [GO:0043318]; positively regulated by positive regulation of cytotoxic T cell degranulation [GO:0043319]